venom-mediated fibrinogenolysis [GO:0044485] (biological process) Also known as: envenomation resulting in fibrinogenolysis in another organism, envenomation resulting in fibrinogenolysis in other organism Relationships: is a type of venom-mediated depletion of circulating fibrinogen [GO:0044536] Definition: A process in which an organism initiates, promotes, or enhances fibrinogenolysis in another organism via the action of a venom. Fibrinogenolysis is the degradation of fibrinogen by proteolytic cleavage. References: PMID:17433397, PMID:17544404 Sources: GOC:fj